{
  "gene": "UniProtKB:Q96GY0",
  "term_id": "UNKNOWN:0002",
  "term_label": "Unknown biological process",
  "gene_name": "Zinc finger C2HC domain-containing protein 1A",
  "gene_symbol": "ZC2HC1A"
}